{
  "gene_name": "Polyubiquitin-C",
  "gene_symbol": "UBC",
  "gene": "UniProtKB:P0CG48",
  "term_id": "GO:0022626",
  "term_label": "cytosolic ribosome"
}